phenol 2-monooxygenase activity [GO:0018662] (molecular function) Sources: EC:1.14.13.7 Also known as: phenol hydroxylase activity, phenol o-hydroxylase activity, phenol,NADPH:oxygen oxidoreductase (2-hydroxylating) Definition: Catalysis of the reaction: phenol + NADPH + H+ + O2 = catechol + NADP+ + H2O. Relationships: is a type of oxidoreductase activity, acting on paired donors, with incorporation or reduction of molecular oxygen, NAD(P)H as one donor, and incorporation of one atom of oxygen [GO:0016709]